protein decanoylation [GO:0051366] (biological process) Also known as: protein amino acid decanoylation Definition: The modification of a protein amino acid by formation of an ester or amide with decanoic acid. Sources: GOC:jsg Relationships: is a type of GO:0006497; is a type of protein acylation [GO:0043543]